methotrexate transport [GO:0051958] (biological process) Definition: The directed movement of methotrexate, 4-amino-10-methylformic acid, into, out of or within a cell, or between cells, by means of some agent such as a transporter or pore. Methotrexate is a folic acid analogue and a potent competitive inhibitor of dihydrofolate reductase. Sources: GOC:ai Relationships: is a type of GO:0006835; is a type of amide transport [GO:0042886]